{
  "gene_name": "Olfactory receptor 52N2",
  "term_id": "GO:0005886",
  "gene_symbol": "OR52N2",
  "gene": "UniProtKB:Q8NGI0",
  "term_label": "plasma membrane"
}